{
  "gene": "UniProtKB:Q6UWP7",
  "term_id": "GO:0016746",
  "gene_name": "Lysocardiolipin acyltransferase 1",
  "term_label": "acyltransferase activity",
  "gene_symbol": "LCLAT1"
}